glucan endo-1,6-beta-glucosidase activity [GO:0046557] (molecular function) Sources: EC:3.2.1.75 Definition: Catalysis of the random hydrolysis of (1->6) linkages in (1->6)-beta-D-glucans. Also known as: endo-(1,6)-beta-D-glucanase activity, 1,6-beta-D-glucan glucanohydrolase activity, beta-1,6-glucan 6-glucanohydrolase activity, beta-1,6-glucan hydrolase activity, beta-1,6-glucanase activity, beta-1,6-glucanase-pustulanase activity, beta-1->6-glucan hydrolase activity, endo-(1->6)-beta-D-glucanase activity, endo-1,6-beta-D-glucanase activity, endo-1,6-beta-glucanase activity, endo-beta-1,6-glucanase activity Relationships: is a type of beta-glucosidase activity [GO:0008422]